{
  "term_id": "UNKNOWN:0002",
  "gene": "UniProtKB:P26371",
  "gene_name": "Keratin-associated protein 5-9",
  "term_label": "Unknown biological process",
  "gene_symbol": "KRTAP5-9"
}